{
  "term_label": "RNA polymerase II transcription regulatory region sequence-specific DNA binding",
  "gene": "UniProtKB:Q96MU6",
  "gene_name": "Zinc finger protein 778",
  "gene_symbol": "ZNF778",
  "term_id": "GO:0000977"
}